{
  "gene_symbol": "HES3",
  "gene_name": "Transcription factor HES-3",
  "term_id": "GO:0000122",
  "term_label": "negative regulation of transcription by RNA polymerase II",
  "gene": "UniProtKB:Q5TGS1"
}